{
  "gene_name": "Putative protein-lysine deacylase ABHD14B",
  "gene_symbol": "ABHD14B",
  "gene": "UniProtKB:Q96IU4",
  "term_label": "hydrolase activity",
  "term_id": "GO:0016787"
}